galactarate catabolic process [GO:0046392] (biological process) Definition: The chemical reactions and pathways resulting in the breakdown of galactarate, the anion of galactaric acid. Relationships: is a type of aldaric acid catabolic process [GO:0019579]; is a type of galactarate metabolic process [GO:0019580] Also known as: galactarate breakdown, galactarate catabolism, galactarate degradation, D-galactarate breakdown, D-galactarate catabolic process, D-galactarate catabolism, D-galactarate degradation Sources: GOC:ai, GOC:pr